aspartate-tRNA ligase activity [GO:0004815] (molecular function) Also known as: aspartyl-tRNA synthetase activity, L-aspartate:tRNAAsp ligase (AMP-forming), aspartic acid translase activity, aspartyl ribonucleate synthetase activity, aspartyl ribonucleic synthetase activity, aspartyl-transfer RNA synthetase activity, aspartyl-transfer ribonucleic acid synthetase activity Definition: Catalysis of the reaction: ATP + L-aspartate + tRNA(Asp) = AMP + diphosphate + L-aspartyl-tRNA(Asp). Sources: EC:6.1.1.12 Relationships: is a type of aminoacyl-tRNA ligase activity [GO:0004812]